ESCRT II complex [GO:0000814] (cellular component) Definition: An endosomal sorting complex required for transport and functions downstream of ESCRT I complex. It consists of the class E vacuolar protein sorting (Vps) proteins and is required for the membrane recruitment of ESCRT III complex and binds to ubiquitinated cargoes. References: PMID:12892785, PMID:12900393 Sources: GOC:rb Also known as: endosomal sorting complex required for transport Relationships: is a type of ESCRT complex [GO:0036452]; is a type of membrane protein complex [GO:0098796]; is part of endosome membrane [GO:0010008]